SCF ubiquitin ligase complex binding [GO:1905761] (molecular function) References: PMID:19723762 Sources: GOC:TermGenie, GOC:dph, GOC:ha Relationships: is a type of protein-containing complex binding [GO:0044877] Also known as: CDL1 complex binding, CRL1 complex binding, Cul1-RING ubiquitin ligase complex binding, SCF complex binding, Skp1/Cul1/F-box protein complex binding, cullin-RING ligase 1 binding, SCF complex substrate recognition subunit binding Definition: Binding to a SCF ubiquitin ligase complex.